laminin binding [GO:0043236] (molecular function) Also known as: laminin-2 binding, laminin-4 binding Relationships: is_a protein binding [GO:0005515]; is a type of extracellular matrix binding [GO:0050840] Subtypes: laminin-1 binding [GO:0043237], laminin binding involved in cell-matrix adhesion [GO:0098638] Sources: GOC:ecd Definition: Binding to a laminin, a major glycoprotein constituent of the basement membrane of cells.